osmosensor activity [GO:0005034] (molecular function) Sources: GOC:dph, GOC:tb Definition: Sensing extracellular osmolarity to initiate a change in cell activity, and spanning the membrane of the cell. Subtypes: GO:1990760 Relationships: is_a GO:0004888; is a type of molecular sensor activity [GO:0140299]